{
  "term_id": "UNKNOWN:0001",
  "term_label": "Unknown molecular function",
  "gene_symbol": "CD101",
  "gene": "UniProtKB:Q93033",
  "gene_name": "Immunoglobulin superfamily member 2"
}